{
  "gene": "UniProtKB:Q96JN2",
  "term_id": "UNKNOWN:0001",
  "gene_name": "Coiled-coil domain-containing protein 136",
  "gene_symbol": "CCDC136",
  "term_label": "Unknown molecular function"
}